{
  "gene_name": "Putative olfactory receptor 1F2",
  "term_id": "GO:0005886",
  "gene_symbol": "OR1F2P",
  "term_label": "plasma membrane",
  "gene": "UniProtKB:Q96R84"
}